negative regulation of sprouting angiogenesis [GO:1903671] (biological process) References: PMID:16756958 Sources: GOC:TermGenie, GO_REF:0000058 Also known as: down regulation of sprouting angiogenesis, down-regulation of sprouting angiogenesis, downregulation of sprouting angiogenesis, inhibition of sprouting angiogenesis Subtypes: negative regulation of cell adhesion involved in sprouting angiogenesis [GO:0106089] Relationships: is a type of negative regulation of angiogenesis [GO:0016525]; is a type of GO:1903670; negatively regulates sprouting angiogenesis [GO:0002040] Definition: Any process that stops, prevents or reduces the frequency, rate or extent of sprouting angiogenesis.